4-(trimethylammonio)butanoate transmembrane transporter activity [GO:1901236] (molecular function) Relationships: is a type of GO:0015651; is a type of GO:0072349 Subtypes: (R)-carnitine:4-(trimethylammonio)butanoate antiporter activity [GO:0044667] References: PMID:16952940, PMID:21784948 Sources: GOC:TermGenie Definition: Enables the transfer of 4-(trimethylammonio)butanoate from one side of a membrane to the other.